thyrotropin-releasing hormone binding [GO:0051449] (molecular function) Relationships: is a type of GO:0017046 Also known as: thyrotropin releasing hormone binding Sources: GOC:ai Definition: Binding to thyrotropin-releasing hormone, a tripeptide hormone that stimulates the release of thyroid-stimulating hormone (TSH) and prolactin by the anterior pituitary and it is produced by the hypothalamus and travels across the median eminence to the pituitary via the pituitary portal system.